{
  "term_label": "regulation of mitochondrial ATP synthesis coupled proton transport",
  "gene": "UniProtKB:Q9BQD7",
  "gene_name": "Adenine nucleotide translocase lysine N-methyltransferase",
  "term_id": "GO:1905706",
  "gene_symbol": "ANTKMT"
}